{
  "gene": "UniProtKB:Q2T9K0",
  "term_id": "UNKNOWN:0003",
  "term_label": "Unknown cellular component",
  "gene_symbol": "TMEM44",
  "gene_name": "Transmembrane protein 44"
}